{
  "term_id": "GO:0097503",
  "gene_name": "Beta-galactoside alpha-2,6-sialyltransferase 1",
  "term_label": "sialylation",
  "gene_symbol": "ST6GAL1",
  "gene": "UniProtKB:P15907"
}